{
  "gene": "UniProtKB:O95183",
  "gene_name": "Vesicle-associated membrane protein 5",
  "term_label": "plasma membrane",
  "gene_symbol": "VAMP5",
  "term_id": "GO:0005886"
}